glutathione oxidase activity [GO:0047950] (molecular function) Sources: EC:1.8.3.3, RHEA:24112 Relationships: is a type of GO:0016670 Also known as: glutathione:oxygen oxidoreductase activity Definition: Catalysis of the reaction: 2 glutathione + O2 = glutathione disulfide + H2O2.